{
  "term_label": "positive regulation of cell population proliferation",
  "gene": "UniProtKB:P11362",
  "gene_symbol": "FGFR1",
  "gene_name": "Fibroblast growth factor receptor 1",
  "term_id": "GO:0008284"
}